{
  "gene_name": "Cyclin-dependent kinase inhibitor 1B",
  "term_id": "GO:0051087",
  "gene_symbol": "CDKN1B",
  "gene": "UniProtKB:P46527",
  "term_label": "protein-folding chaperone binding"
}